{
  "gene_symbol": "SUPT20HL1",
  "term_label": "transcription coregulator activity",
  "gene": "UniProtKB:Q3ZLR7",
  "term_id": "GO:0003712",
  "gene_name": "Transcription factor SPT20 homolog-like 1"
}